{
  "term_label": "Unknown biological process",
  "gene_symbol": "IGFL2",
  "gene_name": "Insulin growth factor-like family member 2",
  "term_id": "UNKNOWN:0002",
  "gene": "UniProtKB:Q6UWQ7"
}